inhibitory extracellular ligand-gated monoatomic ion channel activity [GO:0005237] (molecular function) Subtypes: extracellularly glycine-gated chloride channel activity [GO:0016934] Also known as: inhibitory extracellular ligand-gated ion channel activity Definition: Enables the transmembrane transfer of an ion by a channel that opens when a specific extracellular inhibitory ligand has been bound by the channel complex or one of its constituent parts. Inhibitory ligands, such as GABA or glycine, open chloride-selective channels. Relationships: is a type of extracellular ligand-gated monoatomic ion channel activity [GO:0005230] Sources: GOC:mah, ISBN:0323037070